{
  "gene_symbol": "LHFPL1",
  "term_label": "Unknown molecular function",
  "term_id": "UNKNOWN:0001",
  "gene": "UniProtKB:Q86WI0",
  "gene_name": "LHFPL tetraspan subfamily member 1 protein"
}